{
  "gene": "UniProtKB:Q6NT55",
  "term_label": "Unknown molecular function",
  "gene_symbol": "CYP4F22",
  "gene_name": "Ultra-long-chain fatty acid omega-hydroxylase",
  "term_id": "UNKNOWN:0001"
}